{
  "gene_name": "Keratin-associated protein 1-5",
  "term_label": "Unknown biological process",
  "gene_symbol": "KRTAP1-5",
  "term_id": "UNKNOWN:0002",
  "gene": "UniProtKB:Q9BYS1"
}